{
  "gene": "UniProtKB:P42224",
  "gene_symbol": "STAT1",
  "term_id": "GO:0005634",
  "gene_name": "Signal transducer and activator of transcription 1-alpha_beta",
  "term_label": "nucleus"
}